{
  "term_id": "GO:0008024",
  "term_label": "cyclin/CDK positive transcription elongation factor complex",
  "gene_symbol": "CCNT2",
  "gene_name": "Cyclin-T2",
  "gene": "UniProtKB:O60583"
}